{
  "gene_symbol": "ZNF678",
  "term_id": "UNKNOWN:0003",
  "term_label": "Unknown cellular component",
  "gene": "UniProtKB:Q5SXM1",
  "gene_name": "Zinc finger protein 678"
}